pyrimidine ribonucleoside triphosphate catabolic process [GO:0009210] (biological process) Subtypes: CTP catabolic process [GO:0006254], TTP catabolic process [GO:0046047], UTP catabolic process [GO:0046052] Sources: GOC:go_curators, ISBN:0198506732 Definition: The chemical reactions and pathways resulting in the breakdown of pyrimidine ribonucleoside triphosphate, a compound consisting of a pyrimidine base linked to a ribose sugar esterified with triphosphate on the sugar. Relationships: is a type of pyrimidine nucleoside triphosphate catabolic process [GO:0009149]; is a type of ribonucleoside triphosphate catabolic process [GO:0009203]; is a type of pyrimidine ribonucleoside triphosphate metabolic process [GO:0009208] Also known as: pyrimidine ribonucleoside triphosphate breakdown, pyrimidine ribonucleoside triphosphate catabolism, pyrimidine ribonucleoside triphosphate degradation